{
  "gene": "UniProtKB:Q01851",
  "gene_symbol": "POU4F1",
  "term_label": "RNA polymerase II cis-regulatory region sequence-specific DNA binding",
  "term_id": "GO:0000978",
  "gene_name": "POU domain, class 4, transcription factor 1"
}